hyphal septin ring [GO:0032168] (cellular component) References: PMID:16151244 Sources: GOC:krc, GOC:mah Definition: A tight ring-shaped structure that forms in the division plane within hyphae of filamentous fungi at sites where a septum will form; composed of septins as well as septin-associated proteins. Relationships: is a type of septin ring [GO:0005940]